{
  "gene": "UniProtKB:P43699",
  "term_label": "nucleus",
  "gene_symbol": "NKX2-1",
  "gene_name": "Homeobox protein Nkx-2.1",
  "term_id": "GO:0005634"
}